venom-mediated activation of voltage-gated sodium channel activity [GO:0044494] (BP) Relationships: is a type of venom-mediated perturbation of voltage-gated sodium channel activity [GO:0044492] Definition: A process in which an organism initiates, promotes, or enhances the activity of a voltage-gated sodium channel in another organism via the action of a venom. References: PMID:21781281 Sources: GOC:fj, GOC:jl Also known as: envenomation resulting in positive regulation of voltage-gated sodium channel activity in another organism, envenomation resulting in positive regulation of voltage-gated sodium channel activity in other organism